{
  "gene": "UniProtKB:Q86X51",
  "term_id": "UNKNOWN:0001",
  "gene_symbol": "EZHIP",
  "gene_name": "EZH inhibitory protein",
  "term_label": "Unknown molecular function"
}